positive regulation of keratinocyte migration [GO:0051549] (biological process) Relationships: is a type of positive regulation of epithelial cell migration [GO:0010634]; is a type of regulation of keratinocyte migration [GO:0051547]; positively regulates keratinocyte migration [GO:0051546] Definition: Any process that activates or increases the frequency, rate or extent of keratinocyte migration. Also known as: up regulation of keratinocyte migration, up-regulation of keratinocyte migration, upregulation of keratinocyte migration, activation of keratinocyte migration, stimulation of keratinocyte migration Sources: GOC:ai